{
  "gene_symbol": "FOXM1",
  "gene": "UniProtKB:Q08050",
  "gene_name": "Forkhead box protein M1",
  "term_label": "positive regulation of double-strand break repair",
  "term_id": "GO:2000781"
}